{
  "term_label": "cytoplasm",
  "gene": "UniProtKB:Q8N4E7",
  "term_id": "GO:0005737",
  "gene_symbol": "FTMT",
  "gene_name": "Ferritin, mitochondrial"
}